maltoheptaose transport [GO:2001105] (BP) Sources: GOC:mengo_curators Definition: The directed movement of a maltoheptaoseacetate into, out of or within a cell, or between cells, by means of some agent such as a transporter or pore. Relationships: is a type of GO:2001104 Regulation: RO_0002211 by regulation of maltoheptaose transport [GO:1900306]; negatively regulated by negative regulation of maltoheptaose transport [GO:1900307]; positively regulated by GO:1900308